{
  "gene_symbol": "MIER2",
  "gene_name": "Mesoderm induction early response protein 2",
  "term_id": "GO:0005654",
  "term_label": "nucleoplasm",
  "gene": "UniProtKB:Q8N344"
}